{
  "gene_name": "mRNA export factor GLE1",
  "gene": "UniProtKB:Q53GS7",
  "gene_symbol": "GLE1",
  "term_label": "poly(A)+ mRNA export from nucleus",
  "term_id": "GO:0016973"
}